{
  "term_label": "endoplasmic reticulum",
  "gene": "UniProtKB:Q76MJ5",
  "gene_symbol": "ERN2",
  "term_id": "GO:0005783",
  "gene_name": "Serine_threonine-protein kinase_endoribonuclease IRE2"
}